{
  "term_id": "GO:0045104",
  "gene": "UniProtKB:Q6ZRV2",
  "gene_symbol": "FAM83H",
  "term_label": "intermediate filament cytoskeleton organization",
  "gene_name": "Protein FAM83H"
}